{
  "gene": "UniProtKB:P48023",
  "gene_symbol": "FASLG",
  "gene_name": "Tumor necrosis factor ligand superfamily member 6",
  "term_id": "GO:0008625",
  "term_label": "extrinsic apoptotic signaling pathway via death domain receptors"
}